{
  "gene": "UniProtKB:Q0P6D2",
  "term_label": "Unknown biological process",
  "gene_symbol": "DIPK1C",
  "gene_name": "Divergent protein kinase domain 1C",
  "term_id": "UNKNOWN:0002"
}